TAP complex binding [GO:0062061] (molecular function) References: PMID:17947644 Relationships: is a type of protein-containing complex binding [GO:0044877] Definition: Binding to a TAP complex.